{
  "gene_name": "Hsp90 co-chaperone Cdc37",
  "gene_symbol": "CDC37",
  "gene": "UniProtKB:Q16543",
  "term_label": "protein stabilization",
  "term_id": "GO:0050821"
}